prostaglandin-endoperoxide synthase activity [GO:0004666] (MF) Sources: RHEA:23728 Also known as: (5Z,8Z,11Z,14Z)-icosa-5,8,11,14-tetraenoate,hydrogen-donor:oxygen oxidoreductase activity, (PG)H synthase activity, PG synthetase activity, fatty acid cyclooxygenase activity, prostaglandin G/H synthase activity, prostaglandin endoperoxide synthetase activity, prostaglandin synthase activity, prostaglandin synthetase activity Relationships: is_a GO:0016705 Definition: Catalysis of the reaction: (5Z,8Z,11Z,14Z)-eicosatetraenoate + AH2 + 2 O2 = A + H2O + prostaglandin H2.